{
  "gene": "UniProtKB:Q8IV08",
  "term_label": "Unknown molecular function",
  "gene_symbol": "PLD3",
  "gene_name": "5'-3' exonuclease PLD3",
  "term_id": "UNKNOWN:0001"
}